cyanidin 3-O-[2''-O-(xylosyl)-6''-O-(p-coumaroyl) glucoside] 5-O-glucoside malonyltransferase activity [GO:0102585] (MF) Relationships: is a type of acyltransferase activity, transferring groups other than amino-acyl groups [GO:0016747] Definition: Catalysis of the reaction: anthocyanin A3 + malonyl-CoA = anthocyanin A5 + CoA. References: PMID:17292360 Sources: RHEA:72871